{
  "term_id": "UNKNOWN:0003",
  "term_label": "Unknown cellular component",
  "gene_symbol": "PGBD3",
  "gene": "UniProtKB:Q8N328",
  "gene_name": "PiggyBac transposable element-derived protein 3"
}